{
  "gene_symbol": "ATG4D",
  "gene_name": "Cysteine protease ATG4D",
  "term_id": "GO:0000423",
  "term_label": "mitophagy",
  "gene": "UniProtKB:Q86TL0"
}